negative regulation of epithelial cell-cell adhesion involved in epithelium migration [GO:1903682] (biological process) Definition: Any process that stops, prevents or reduces the frequency, rate or extent of epithelial cell-cell adhesion involved in epithelium migration. References: PMID:18394891 Sources: GOC:TermGenie, GOC:als, GO_REF:0000058 Relationships: is_a negative regulation of cell-cell adhesion [GO:0022408]; is a type of negative regulation of multicellular organismal process [GO:0051241]; is a type of regulation of epithelial cell-cell adhesion involved in epithelium migration [GO:1903681]; negatively regulates epithelial cell-cell adhesion involved in epithelium migration [GO:0090137] Also known as: down regulation of epithelial cell-cell adhesion involved in epithelium migration, down-regulation of epithelial cell-cell adhesion involved in epithelium migration, downregulation of epithelial cell-cell adhesion involved in epithelium migration, inhibition of epithelial cell-cell adhesion involved in epithelium migration